{
  "gene_name": "Protein FAM90A16",
  "gene": "UniProtKB:P0DV73",
  "term_label": "Unknown biological process",
  "gene_symbol": "FAM90A16",
  "term_id": "UNKNOWN:0002"
}